{
  "term_label": "Unknown biological process",
  "term_id": "UNKNOWN:0002",
  "gene": "UniProtKB:Q8N239",
  "gene_name": "Kelch-like protein 34",
  "gene_symbol": "KLHL34"
}